{
  "gene_name": "Placenta-specific protein 9",
  "term_id": "UNKNOWN:0002",
  "gene_symbol": "PLAC9",
  "term_label": "Unknown biological process",
  "gene": "UniProtKB:Q5JTB6"
}